{
  "gene": "UniProtKB:O43660",
  "gene_symbol": "PLRG1",
  "term_label": "Prp19 complex",
  "gene_name": "Pleiotropic regulator 1",
  "term_id": "GO:0000974"
}